{
  "term_label": "cell chemotaxis",
  "term_id": "GO:0060326",
  "gene": "UniProtKB:P0DP73",
  "gene_name": "Beta-defensin 130B",
  "gene_symbol": "DEFB130B"
}